{
  "gene_symbol": "RTL10",
  "gene": "UniProtKB:Q7L3V2",
  "gene_name": "Protein Bop",
  "term_label": "mitochondrion",
  "term_id": "GO:0005739"
}